{
  "gene": "UniProtKB:Q8NEM2",
  "gene_name": "SHC SH2 domain-binding protein 1",
  "gene_symbol": "SHCBP1",
  "term_id": "UNKNOWN:0001",
  "term_label": "Unknown molecular function"
}